{
  "term_id": "GO:0051209",
  "gene": "UniProtKB:P28335",
  "term_label": "release of sequestered calcium ion into cytosol",
  "gene_symbol": "HTR2C",
  "gene_name": "5-hydroxytryptamine receptor 2C"
}